phospholipase C-activating opsin-mediated signaling pathway [GO:0030265] (biological process) Definition: A phospholipase C-activating receptor G protein-coupled receptor signaling pathway that starts with an opsin being activated by a photon, and transmitting the signal through the Gq-mediated activation of phospholipase C (PLC). PLC hydrolyses phosphatidylinositol 4,5-bisphosphate (PIP2) into the second messengers inositol-1,4,5,-triphosphate (IP3) and diacylglycerol (DAG). The second messengers, including cGMP, activate channels that result in transmission of the light signal  through the synapses. Typical examples are rhabdomeric photoreceptors in the eyes of protostomes. References: PMID:19720651, PMID:22498302, PMID:8823931 Also known as: PLC-activating rhodopsin mediated signaling pathway, phospholipase C-activating rhodopsin mediated G-protein coupled receptor signaling pathway, phospholipase C-activating rhodopsin mediated signaling pathway, rhodopsin mediated G protein signaling, coupled to IP3 second messenger, rhodopsin mediated G protein signalling, coupled to IP3 second messenger, rhodopsin mediated G-protein signaling, coupled to IP3 second messenger, rhodopsin mediated G-protein signalling, coupled to IP3 second messenger Relationships: is_a phospholipase C-activating G protein-coupled receptor signaling pathway [GO:0007200]; is a type of GO:0016056; has part phospholipase C activity [GO:0004629] Regulation: RO_0002212 by negative regulation of phospholipase C-activating phototransduction signaling pathway [GO:0016060]